{
  "gene_symbol": "RANBP3",
  "gene": "UniProtKB:Q9H6Z4",
  "gene_name": "Ran-binding protein 3",
  "term_id": "GO:0005643",
  "term_label": "nuclear pore"
}